{
  "gene_name": "Putative inactive group IIC secretory phospholipase A2",
  "gene": "UniProtKB:Q5R387",
  "gene_symbol": "PLA2G2C",
  "term_id": "GO:0005102",
  "term_label": "signaling receptor binding"
}